{
  "term_id": "UNKNOWN:0002",
  "term_label": "Unknown biological process",
  "gene_name": "Endogenous retrovirus group FC1 member 1 Env polyprotein",
  "gene": "UniProtKB:P60608",
  "gene_symbol": "ERVFC1-1"
}